{
  "term_id": "GO:0007399",
  "gene_symbol": "SRGAP2",
  "term_label": "nervous system development",
  "gene": "UniProtKB:O75044",
  "gene_name": "SLIT-ROBO Rho GTPase-activating protein 2"
}